{
  "term_id": "GO:0006264",
  "gene_name": "DNA polymerase subunit gamma-1",
  "gene": "UniProtKB:P54098",
  "gene_symbol": "POLG",
  "term_label": "mitochondrial DNA replication"
}